{
  "gene_name": "Protein DENND6B",
  "gene": "UniProtKB:Q8NEG7",
  "gene_symbol": "DENND6B",
  "term_id": "GO:0055037",
  "term_label": "recycling endosome"
}